L-arginine catabolic process to succinate [GO:0019545] (biological process) Sources: GOC:go_curators Definition: The chemical reactions and pathways resulting in the breakdown of L-arginine into other compounds, including succinate. Relationships: is a type of succinate metabolic process [GO:0006105]; is a type of L-arginine catabolic process [GO:0006527] Also known as: arginine breakdown to succinate, arginine degradation to succinate